{
  "gene_name": "Kunitz-type protease inhibitor 4",
  "gene_symbol": "SPINT4",
  "term_id": "UNKNOWN:0001",
  "term_label": "Unknown molecular function",
  "gene": "UniProtKB:Q6UDR6"
}